abscisic acid homeostasis [GO:1902265] (BP) Definition: Any process involved in the maintenance of an internal steady state of abscisic acid within an organism or cell. References: PMID:23252460 Sources: GOC:TermGenie Also known as: 2-cis-abscisate homeostasis, ABA homeostasis Relationships: is_a lipid homeostasis [GO:0055088] Subtypes: intracellular abscisic acid homeostasis [GO:1902266]